L-methionine catabolic process to 3-methylthiopropanoate [GO:0000954] (biological process) Relationships: is a type of amino acid catabolic process to carboxylic acid via Ehrlich pathway [GO:0000948]; is_a fatty acid biosynthetic process [GO:0006633]; is a type of L-methionine catabolic process [GO:0009087]; is a type of sulfur compound biosynthetic process [GO:0044272] Definition: The chemical reactions and pathways involving the catabolism of amino acids to produce carboxylic acids with one carbon less than the starting amino acid. In S. cerevisiae, this is known to occur for leucine, isoleucine, valine, methionine, phenylalanine, tyrosine, or tryptophan. When L-methionine is used as the substrate, 3-methylthiopropanoate is produced. Often referred to as the Ehrlich pathway, these reactions generally occur during fermentation to produce a variety of carboxylic acids, sometimes collectively referred to as fusel acids. Depending on the redox state of the cells, alcohol derivatives may be produced instead of carboxylic acids. References: PMID:18281432 Sources: GOC:krc